wound healing, spreading of epidermal cells [GO:0035313] (biological process) Regulation: regulated by regulation of wound healing, spreading of epidermal cells [GO:1903689]; negatively regulated by negative regulation of wound healing, spreading of epidermal cells [GO:1903690]; positively regulated by positive regulation of wound healing, spreading of epidermal cells [GO:1903691] Relationships: is a type of wound healing, spreading of cells [GO:0044319] References: PMID:15269788 Sources: GOC:bf Definition: The migration of an epidermal cell along or through a wound gap that contributes to the reestablishment of a continuous epidermis.